nucleate erythrocyte maturation [GO:0043362] (biological process) Also known as: nucleate RBC maturation, nucleate red blood cell maturation Definition: A developmental process, independent of morphogenetic (shape) change, that is required for a nucleate erythrocyte to attain its fully functional state. A nucleate erythrocyte is an erythrocyte with a nucleus. Relationships: is_a erythrocyte maturation [GO:0043249]; is part of GO:0048823 Sources: GOC:devbiol, GOC:jl